{
  "term_label": "negative regulation of blood pressure",
  "term_id": "GO:0045776",
  "gene": "UniProtKB:P29475",
  "gene_symbol": "NOS1",
  "gene_name": "Nitric oxide synthase 1"
}